oligosaccharide reducing-end xylanase activity [GO:0033951] (molecular function) Also known as: Rex, beta-D-xylopyranosyl-(1->4)-beta-D-xylopyranosyl-(1->4)-beta-D-xylopyranose reducing-end xylanase activity, reducing end xylose-releasing exo-oligoxylanase activity Definition: Catalysis of the hydrolysis of 1,4-beta-D-xylose residues from the reducing end of oligosaccharides. Sources: EC:3.2.1.156 Relationships: is a type of GO:0004553